pyruvate dehydrogenase (NADP+) activity [GO:0050243] (molecular function) Relationships: is a type of oxidoreductase activity, acting on the aldehyde or oxo group of donors, NAD or NADP as acceptor [GO:0016620] Definition: Catalysis of the reaction: CoA + NADP+ + pyruvate = acetyl-CoA + CO2 + NADPH. Sources: RHEA:17425 Also known as: pyruvate:NADP(+) oxidoreductase activity, pyruvate:NADP+ 2-oxidoreductase (CoA-acetylating), pyruvate:NADP+ oxidoreductase activity